{
  "gene_symbol": "H3Y2",
  "gene": "UniProtKB:P0DPK5",
  "gene_name": "Histone H3.X",
  "term_label": "nucleosome",
  "term_id": "GO:0000786"
}